{
  "gene_name": "Protein DEK",
  "term_id": "GO:2000779",
  "gene_symbol": "DEK",
  "gene": "UniProtKB:P35659",
  "term_label": "regulation of double-strand break repair"
}